negative regulation of red or far-red light signaling pathway [GO:0090229] (biological process) Definition: Any process that decreases the rate, frequency or extent of the red or far-red signaling pathway, the series of molecular signals initiated upon sensing by photoreceptor molecules of red light or far red light. Also known as: negative regulation of phytochrome signaling pathway, negative regulation of red or far-red light signalling pathway Relationships: is_a negative regulation of signal transduction [GO:0009968]; is a type of regulation of red or far-red light signaling pathway [GO:0090227]; negatively regulates GO:0010017 Sources: GOC:tb